{
  "term_label": "DNA-binding transcription factor activity, RNA polymerase II-specific",
  "gene_symbol": "ZSCAN31",
  "term_id": "GO:0000981",
  "gene": "UniProtKB:Q96LW9",
  "gene_name": "Zinc finger and SCAN domain-containing protein 31"
}